acetate transport [GO:0006846] (biological process) Definition: The directed movement of acetate into, out of or within a cell, or between cells, by means of some agent such as a transporter or pore. Sources: GOC:krc Relationships: is a type of monocarboxylic acid transport [GO:0015718] Subtypes: acetate transmembrane transport [GO:0035433]